{
  "term_label": "Unknown cellular component",
  "term_id": "UNKNOWN:0003",
  "gene_symbol": "A8MWP4",
  "gene_name": "Putative uncharacterized protein ENSP00000401716",
  "gene": "UniProtKB:A8MWP4"
}